{
  "term_id": "GO:0005634",
  "gene_name": "Protein IWS1 homolog",
  "gene_symbol": "IWS1",
  "term_label": "nucleus",
  "gene": "UniProtKB:Q96ST2"
}